corticotropin receptor activity [GO:0004978] (molecular function) Also known as: ACTH receptor activity, adrenocorticotropic hormone receptor activity, adrenocorticotropin receptor activity Relationships: is a type of melanocortin receptor activity [GO:0004977]; is a type of neuropeptide receptor activity [GO:0008188]; has part GO:0042562 Definition: Combining with corticotropin to initiate a change in cell activity. Sources: GOC:ai